{
  "term_id": "UNKNOWN:0001",
  "gene": "UniProtKB:Q96BW5",
  "term_label": "Unknown molecular function",
  "gene_symbol": "PTER",
  "gene_name": "Phosphotriesterase-related protein"
}